{
  "term_label": "protein transmembrane transporter activity",
  "term_id": "GO:0008320",
  "gene_name": "Mitochondrial import inner membrane translocase subunit Tim23",
  "gene": "UniProtKB:O14925",
  "gene_symbol": "TIMM23"
}